{
  "term_id": "GO:0098919",
  "gene": "UniProtKB:Q9HCD6",
  "term_label": "structural constituent of postsynaptic density",
  "gene_symbol": "TANC2",
  "gene_name": "Protein TANC2"
}